{
  "term_label": "Arp2/3 complex-mediated actin nucleation",
  "gene_name": "WAS_WASL-interacting protein family member 3",
  "gene": "UniProtKB:A6NGB9",
  "term_id": "GO:0034314",
  "gene_symbol": "WIPF3"
}